Smp focus [GO:0062238] (cellular component) References: PMID:22582262, PMID:31811152 Relationships: is a type of nuclear protein-containing complex [GO:0140513]; is a type of ribonucleoprotein complex [GO:1990904]; is part of nuclear chromosome [GO:0000228] Definition: A DNA-binding ribonucleoprotein complex that contains a lncRNA complementary to the bound chromosomal locus and is involved in the tethering homologous chromosomes together during chromosome pairing at meiotic prophase I. Also known as: Smp dot